regulation of nematode pharynx morphogenesis [GO:0110041] (biological process) Subtypes: negative regulation of nematode pharynx morphogenesis [GO:0110042], positive regulation of nematode pharynx morphogenesis [GO:0110043] References: PMID:20805556 Sources: GOC:rz Relationships: is a type of regulation of animal organ morphogenesis [GO:2000027]; regulates nematode pharynx morphogenesis [GO:0110040] Definition: Any process that modulates the frequency, rate or extent of nematode pharynx morphogenesis, the process in which the anatomical structure of the pharynx is generated and organized.